{
  "term_id": "GO:0003682",
  "gene_symbol": "MBD5",
  "gene": "UniProtKB:Q9P267",
  "term_label": "chromatin binding",
  "gene_name": "Methyl-CpG-binding domain protein 5"
}